mRNA export from nucleus [GO:0006406] (BP) Also known as: mRNA export from cell nucleus, mRNA export out of nucleus, mRNA transport from nucleus to cytoplasm, mRNA-nucleus export Definition: The directed movement of mRNA from the nucleus to the cytoplasm. Subtypes: GO:0016973, GO:0031990 Regulation: regulated by GO:0010793 Sources: GOC:ma Relationships: is a type of RNA export from nucleus [GO:0006405]; is a type of GO:0051028; is part of gene expression [GO:0010467]